{
  "gene_symbol": "APLP1",
  "term_id": "GO:0005886",
  "term_label": "plasma membrane",
  "gene": "UniProtKB:P51693",
  "gene_name": "Amyloid beta precursor like protein 1"
}